{
  "term_label": "catecholamine catabolic process",
  "gene_symbol": "TOMT",
  "term_id": "GO:0042424",
  "gene_name": "Transmembrane O-methyltransferase",
  "gene": "UniProtKB:Q8WZ04"
}